{
  "term_id": "UNKNOWN:0003",
  "gene_name": "PLAC8-like protein 1",
  "gene_symbol": "PLAC8L1",
  "gene": "UniProtKB:A1L4L8",
  "term_label": "Unknown cellular component"
}